positive regulation of nuclear division [GO:0051785] (biological process) Definition: Any process that activates or increases the frequency, rate or extent of nuclear division, the partitioning of the nucleus and its genetic information. Sources: GOC:ai Also known as: up regulation of nuclear division, up-regulation of nuclear division, upregulation of nuclear division, activation of nuclear division, stimulation of nuclear division Relationships: is a type of positive regulation of organelle organization [GO:0010638]; is a type of GO:0051783; positively regulates nuclear division [GO:0000280] Subtypes: GO:0045836, positive regulation of mitotic nuclear division [GO:0045840]